neuronal dense core vesicle membrane [GO:0099012] (cellular component) Definition: The lipid bilayer surrounding a neuronal dense core vesicle. Sources: GOC:dos Relationships: is a type of GO:0032127; is part of neuronal dense core vesicle [GO:0098992]